{
  "gene_name": "C-type lectin domain family 12 member B",
  "gene": "UniProtKB:Q2HXU8",
  "gene_symbol": "CLEC12B",
  "term_id": "GO:0009897",
  "term_label": "external side of plasma membrane"
}